{
  "term_id": "GO:0004842",
  "gene": "UniProtKB:Q8WVD5",
  "gene_symbol": "RNF141",
  "gene_name": "RING finger protein 141",
  "term_label": "ubiquitin-protein transferase activity"
}